{
  "term_id": "UNKNOWN:0002",
  "gene": "UniProtKB:Q2TB10",
  "term_label": "Unknown biological process",
  "gene_symbol": "ZNF800",
  "gene_name": "Zinc finger protein 800"
}